{
  "gene_name": "Tumor necrosis factor receptor superfamily member 13B",
  "term_label": "negative regulation of B cell proliferation",
  "gene": "UniProtKB:O14836",
  "gene_symbol": "TNFRSF13B",
  "term_id": "GO:0030889"
}